RNA NAD+-cap (NAD+-forming) hydrolase activity [GO:0110152] (molecular function) Definition: Catalysis of the reaction: a 5'-end NAD+-phospho-ribonucleoside in mRNA + H2O = a 5'-end phospho-ribonucleoside in mRNA + H+ + NAD+. Also known as: RNA NAD-cap (NAD-forming) hydrolase activity Note: This reaction specifically hydrolyzes the nicotinamide adenine dinucleotide (NAD) cap from a subset of RNAs by removing the entire NAD moiety from the 5'-end of an NAD-capped RNA. Relationships: is a type of hydrolase activity, acting on acid anhydrides, in phosphorus-containing anhydrides [GO:0016818]; is a type of catalytic activity, acting on RNA [GO:0140098] References: PMID:28283058 Sources: GOC:sp, RHEA:60880